{
  "term_label": "DNA-binding transcription factor activity, RNA polymerase II-specific",
  "gene_symbol": "ZEB1",
  "gene": "UniProtKB:P37275",
  "gene_name": "Zinc finger E-box-binding homeobox 1",
  "term_id": "GO:0000981"
}